{
  "gene_symbol": "IQUB",
  "gene_name": "IQ and ubiquitin-like domain-containing protein",
  "term_id": "UNKNOWN:0001",
  "term_label": "Unknown molecular function",
  "gene": "UniProtKB:Q8NA54"
}